{
  "gene": "UniProtKB:A6NDN8",
  "gene_symbol": "A6NDN8",
  "term_label": "Unknown biological process",
  "term_id": "UNKNOWN:0002",
  "gene_name": "Putative ubiquitin-like protein FUBI-like protein ENSP00000310146"
}